ribose phosphate metabolic process [GO:0019693] (biological process) Subtypes: ribonucleotide metabolic process [GO:0009259], GO:0046390, GO:0046391, D-ribose 5-phosphate catabolic process [GO:1901279] Definition: The chemical reactions and pathways involving ribose phosphate, any phosphorylated ribose sugar. Relationships: is a type of phosphate-containing compound metabolic process [GO:0006796]; is a type of GO:0019637; is a type of carbohydrate derivative metabolic process [GO:1901135] Sources: GOC:ai Also known as: ribose phosphate metabolism